{
  "gene_symbol": "CCR5",
  "term_id": "GO:0019722",
  "term_label": "calcium-mediated signaling",
  "gene": "UniProtKB:P51681",
  "gene_name": "C-C chemokine receptor type 5"
}